{
  "gene_symbol": "CXCL8",
  "gene": "UniProtKB:P10145",
  "gene_name": "Interleukin-8",
  "term_label": "chemokine activity",
  "term_id": "GO:0008009"
}